2,3-dimethylmalate lyase activity [GO:0047529] (molecular function) Sources: EC:4.1.3.32, RHEA:10472 Also known as: (2R,3S)-2,3-dimethylmalate pyruvate-lyase (propanoate-forming), (2R,3S)-2,3-dimethylmalate pyruvate-lyase activity, 2,3-dimethylmalate pyruvate-lyase activity Relationships: is a type of oxo-acid-lyase activity [GO:0016833] Definition: Catalysis of the reaction: (2R,3S)-2,3-dimethylmalate = propanoate + pyruvate.